negative regulation of pancreatic trypsinogen secretion [GO:1904243] (biological process) Also known as: down regulation of pancreatic trypsinogen release, down regulation of pancreatic trypsinogen secretion, down-regulation of pancreatic trypsinogen release, down-regulation of pancreatic trypsinogen secretion, downregulation of pancreatic trypsinogen release, downregulation of pancreatic trypsinogen secretion, negative regulation of pancreatic trypsinogen release, inhibition of pancreatic trypsinogen release, inhibition of pancreatic trypsinogen secretion Relationships: is a type of negative regulation of protein secretion [GO:0050709]; is a type of GO:1904242; negatively regulates GO:1990747 References: PMID:12771515 Sources: GOC:TermGenie, GO_REF:0000058 Definition: Any process that stops, prevents or reduces the frequency, rate or extent of pancreatic trypsinogen secretion.